unidimensional cell growth [GO:0009826] (biological process) Regulation: regulated by regulation of unidimensional cell growth [GO:0051510]; negatively regulated by GO:0051511; positively regulated by positive regulation of unidimensional cell growth [GO:0051512] Also known as: cell growth along one axis, cell growth in one dimension, cell morphogenesis by unidimensional growth, polar cell growth, polarized cell growth, cell elongation Subtypes: dorsal closure, elongation of leading edge cells [GO:0007394], cell tip growth [GO:0009932], monopolar cell growth [GO:0042814], GO:0042815, zygote elongation [GO:0080159], cell elongation involved in imaginal disc-derived wing morphogenesis [GO:0090254], seed trichome elongation [GO:0090378] Note: Unidimensional cell growth refers to a change in both cell size and cell shape. For cell shape changes where cell size is not affected, consider instead the term 'regulation of cell shape ; GO:0008360' and its children. Definition: The process in which a cell irreversibly increases in size in one [spatial] dimension or along one axis, resulting in the morphogenesis of the cell. Relationships: is a type of cell morphogenesis [GO:0000902]; is a type of cell growth [GO:0016049]; is a type of developmental growth involved in morphogenesis [GO:0060560] Sources: ISBN:0943088399